{
  "term_id": "GO:0006828",
  "gene_symbol": "ATP2C1",
  "gene": "UniProtKB:P98194",
  "gene_name": "Calcium-transporting ATPase type 2C member 1",
  "term_label": "manganese ion transport"
}